{
  "gene_symbol": "IL17RD",
  "term_label": "Unknown biological process",
  "term_id": "UNKNOWN:0002",
  "gene_name": "Interleukin-17 receptor D",
  "gene": "UniProtKB:Q8NFM7"
}